protein kinase C binding [GO:0005080] (molecular function) Relationships: is a type of GO:0019901 Sources: GOC:jl Definition: Binding to protein kinase C. Also known as: PKC alpha binding, PKC binding, PKC delta binding, PKC eta binding, protein kinase C alpha binding, protein kinase C delta binding, protein kinase C eta binding